{
  "term_id": "GO:0000467",
  "gene_symbol": "EXOSC8",
  "gene_name": "Exosome complex component RRP43",
  "gene": "UniProtKB:Q96B26",
  "term_label": "exonucleolytic trimming to generate mature 3'-end of 5.8S rRNA from tricistronic rRNA transcript (SSU-rRNA, 5.8S rRNA, LSU-rRNA)"
}